{
  "gene_name": "Cyclic GMP-AMP synthase",
  "term_label": "positive regulation of type I interferon production",
  "term_id": "GO:0032481",
  "gene_symbol": "CGAS",
  "gene": "UniProtKB:Q8N884"
}